{
  "term_label": "3alpha,7alpha,12alpha-trihydroxy-5beta-cholestanoyl-CoA 24-hydroxylase activity",
  "gene": "UniProtKB:Q99424",
  "gene_symbol": "ACOX2",
  "gene_name": "Peroxisomal acyl-coenzyme A oxidase 2",
  "term_id": "GO:0033791"
}